{
  "gene_name": "Regucalcin",
  "gene": "UniProtKB:Q15493",
  "gene_symbol": "RGN",
  "term_label": "Unknown cellular component",
  "term_id": "UNKNOWN:0003"
}